{
  "gene_symbol": "UTP3",
  "gene_name": "Something about silencing protein 10",
  "gene": "UniProtKB:Q9NQZ2",
  "term_label": "maturation of SSU-rRNA from tricistronic rRNA transcript (SSU-rRNA, 5.8S rRNA, LSU-rRNA)",
  "term_id": "GO:0000462"
}